{
  "gene_symbol": "GARIN2",
  "term_id": "UNKNOWN:0003",
  "gene": "UniProtKB:Q8N9W8",
  "gene_name": "Golgi-associated RAB2 interactor protein 2",
  "term_label": "Unknown cellular component"
}